4-hydroxyphenylacetate 1-monooxygenase activity [GO:0018665] (molecular function) Definition: Catalysis of the reaction: 4-hydroxyphenylacetate + NADPH + H+ + O2 = homogentisate + NADP+ + H2O. Also known as: 4-hydroxyphenyl-acetate 1-hydroxylase activity, 4-HPA 1-hydroxylase activity, 4-hydroxyphenylacetate 1-hydroxylase activity, 4-hydroxyphenylacetate,NAD(P)H:oxygen oxidoreductase (1-hydroxylating), 4-hydroxyphenylacetic 1-hydroxylase activity Sources: EC:1.14.13.18 Relationships: is a type of oxidoreductase activity, acting on paired donors, with incorporation or reduction of molecular oxygen, NAD(P)H as one donor, and incorporation of one atom of oxygen [GO:0016709]